growth [GO:0040007] (biological process) Note: See also the biological process term 'cell growth ; GO:0016049'. Definition: The increase in size or mass of an entire organism, a part of an organism or a cell. Also known as: growth pattern, non-developmental growth Sources: GOC:bf, GOC:ma Subtypes: GO:0007117, cell growth [GO:0016049], GO:0030447, developmental growth [GO:0048589], GO:0080189, GO:0080190 Relationships: is a type of biological_process [GO:0008150] Regulation: regulated by regulation of growth [GO:0040008]; negatively regulated by GO:0045926; positively regulated by positive regulation of growth [GO:0045927]